mitochondrial NAD transmembrane transport [GO:1990549] (biological process) References: PMID:16291748 Definition: The process in which NAD is transported across a mitochondrial membrane, into or out of the mitochondrion. Relationships: is_a NAD transmembrane transport [GO:0035352]